{
  "term_id": "GO:0034715",
  "gene_name": "Small nuclear ribonucleoprotein F",
  "gene": "UniProtKB:P62306",
  "term_label": "pICln-Sm protein complex",
  "gene_symbol": "SNRPF"
}